{
  "gene_symbol": "USP16",
  "term_id": "GO:0045893",
  "term_label": "positive regulation of DNA-templated transcription",
  "gene_name": "Ubiquitin carboxyl-terminal hydrolase 16",
  "gene": "UniProtKB:Q9Y5T5"
}